p38MAPK cascade [GO:0038066] (BP) References: PMID:20811974, PMID:23125017, PMID:32794416 Regulation: regulated by GO:1900744; positively regulated by positive regulation of p38MAPK cascade [GO:1900745]; negatively regulated by negative regulation of p38MAPK cascade [GO:1903753] Also known as: p38 MAPK cascade, p38 cascade, osmosensory signaling MAPK cascade, MAPK14 cascade Relationships: is a type of MAPK cascade [GO:0000165] Definition: A MAPK cascade containing at least the p38MAPK (MAPK14) MAP kinase, or Hog1 in yeast. It starts with the activation of a MAP3K, and the consecutive activation of a MPK2K and of p38MAPK. The cascade can also contain an additional tier: the upstream MAP4K. The kinases in each tier phosphorylate and activate the kinases in the downstream tier. The p38MAPK cascade is activated by stress signals, including hyperosmolarity, as well as by G protein-coupled receptors, growth factors, and cytokines, and results in cellular responses such as cell proliferation, cell differentiation, apoptosis and inflammation.